{
  "gene_name": "Inositol polyphosphate 4-phosphatase type II",
  "term_id": "GO:0016316",
  "term_label": "phosphatidylinositol-3,4-bisphosphate 4-phosphatase activity",
  "gene_symbol": "INPP4B",
  "gene": "UniProtKB:O15327"
}